mesaconyl-CoA hydratase activity [GO:0043881] (molecular function) References: PMID:16856935, PMID:16856937 Definition: Catalysis of the hydration of mesaconyl-CoA to beta-methylmalyl-CoA. Relationships: is a type of hydro-lyase activity [GO:0016836] Note: This function is part of an alternate glyoxylate cycle for acetate assimilation. Also known as: beta-methylmalyl-CoA dehydratase activity, mesaconyl-coenzyme A hydratase activity, mch